{
  "gene_symbol": "ITLN2",
  "term_label": "oligosaccharide binding",
  "gene_name": "Intelectin-2",
  "gene": "UniProtKB:Q8WWU7",
  "term_id": "GO:0070492"
}